RNA polymerase II termination complex [GO:0110103] (cellular component) Definition: A conserved protein complex capable of 5'-3' exoribonuclease activity. It is able to promote RNA polymerase II (RNAPII) transcription termination by degrading pre-mRNA from the newly formed 5' phosphorylated end. Also known as: TXT complex Note: In S. cerevisiae, this complex is formed by RAI1 and RAT1; in H. sapiens it is formed by Twi12, Xrn2 and Tan1. References: PMID:23200120, PMID:25722373 Sources: GOC:lnp Relationships: is a type of GO:0140513; is a type of exoribonuclease complex [GO:1905354]